{
  "term_id": "GO:0010008",
  "gene_symbol": "ABHD17A",
  "term_label": "endosome membrane",
  "gene_name": "Alpha_beta hydrolase domain-containing protein 17A",
  "gene": "UniProtKB:Q96GS6"
}